guiding stereospecific synthesis activity [GO:0042349] (molecular function) Also known as: dirigent protein Relationships: is a type of enzyme regulator activity [GO:0030234] Sources: GOC:ma Definition: The orientation of free radical substrates in such a way that only a particular stereoisomer is synthesized by an enzyme. Best characterized as a function during lignan biosynthesis.